{
  "term_id": "GO:0097503",
  "gene_symbol": "C20orf173",
  "gene": "UniProtKB:Q96LM9",
  "term_label": "sialylation",
  "gene_name": "Uncharacterized protein C20orf173"
}